{
  "gene_name": "Serine_threonine-protein kinase N1",
  "gene": "UniProtKB:Q16512",
  "gene_symbol": "PKN1",
  "term_label": "Unknown cellular component",
  "term_id": "UNKNOWN:0003"
}